{
  "gene": "UniProtKB:Q8N141",
  "gene_name": "Zinc finger protein 82 homolog",
  "term_id": "GO:0000981",
  "gene_symbol": "ZFP82",
  "term_label": "DNA-binding transcription factor activity, RNA polymerase II-specific"
}